isoprenoid transport [GO:0046864] (biological process) Subtypes: GO:0046865 Sources: GOC:ai Definition: The directed movement of isoprenoids into, out of or within a cell, or between cells, by means of some agent such as a transporter or pore. Isoprenoids comprise a group of compounds containing or derived from linked isoprene (3-methyl-2-butenylene) residues. Relationships: is a type of lipid transport [GO:0006869]